{
  "gene_symbol": "BEND7",
  "gene_name": "BEN domain-containing protein 7",
  "term_id": "UNKNOWN:0002",
  "gene": "UniProtKB:Q8N7W2",
  "term_label": "Unknown biological process"
}